{
  "gene_name": "Elongation of very long chain fatty acids protein 1",
  "gene": "UniProtKB:Q9BW60",
  "gene_symbol": "ELOVL1",
  "term_id": "GO:0019367",
  "term_label": "fatty acid elongation, saturated fatty acid"
}